cellular response to 2,3,7,8-tetrachlorodibenzodioxine [GO:1904613] (biological process) Definition: Any process that results in a change in state or activity of a cell (in terms of movement, secretion, enzyme production, gene expression, etc.) as a result of a 2,3,7,8-tetrachlorodibenzodioxine stimulus. References: PMID:23196670 Sources: GOC:TermGenie, GO_REF:0000071 Relationships: is a type of GO:0070887; is_a response to 2,3,7,8-tetrachlorodibenzodioxine [GO:1904612] Also known as: cellular response to TCDD, cellular response to dioxin